{
  "gene_name": "Putative homeobox protein Meis3-like 1",
  "gene_symbol": "MEIS3P1",
  "gene": "UniProtKB:A6NDR6",
  "term_id": "GO:0009887",
  "term_label": "animal organ morphogenesis"
}